{
  "term_id": "UNKNOWN:0001",
  "term_label": "Unknown molecular function",
  "gene_name": "Mucin-like protein 3",
  "gene_symbol": "MUCL3",
  "gene": "UniProtKB:Q3MIW9"
}